photoreceptor cell fate commitment [GO:0046552] (biological process) Subtypes: eye photoreceptor cell fate commitment [GO:0042706], ocellus photoreceptor cell fate commitment [GO:0042707] Relationships: is a type of neuron fate commitment [GO:0048663]; is part of photoreceptor cell differentiation [GO:0046530] Sources: GOC:mtg_sensu Definition: The process in which the developmental fate of a cell becomes restricted such that it will develop into a photoreceptor cell. A photoreceptor cell is a cell that responds to incident electromagnetic radiation. Different classes of photoreceptor have different spectral sensitivities and express different photosensitive pigments.